protein binding [GO:0005515] (molecular function) Definition: Binding to a protein. Sources: GOC:go_curators Regulation: negatively regulated by negative regulation of protein binding [GO:0032091]; positively regulated by positive regulation of protein binding [GO:0032092]; RO_0002211 by GO:0043393 Subtypes: SNARE binding [GO:0000149], GO:0001098, GO:0001846, complement binding [GO:0001848], farnesylated protein binding [GO:0001918], G-protein alpha-subunit binding [GO:0001965], fibronectin binding [GO:0001968], p53 binding [GO:0002039], opsin binding [GO:0002046], GO:0002162, signaling receptor binding [GO:0005102], GO:0005516, lamin binding [GO:0005521], profilin binding [GO:0005522], beta-catenin binding [GO:0008013], cytoskeletal protein binding [GO:0008092], transcription factor binding [GO:0008134], poly-glutamine tract binding [GO:0008267], phytochrome binding [GO:0010313], Wnt-protein binding [GO:0017147], growth factor binding [GO:0019838], GO:0019899, protein domain specific binding [GO:0019904], cytokine binding [GO:0019955], clathrin binding [GO:0030276], cyclin binding [GO:0030332], hemoglobin binding [GO:0030492], GTP-dependent protein binding [GO:0030742], beta-2-microglobulin binding [GO:0030881], GO:0030984, heat shock protein binding [GO:0031072], denatured protein binding [GO:0031249], GO:0031369, hexon binding [GO:0031423], GO:0031681, G-protein gamma-subunit binding [GO:0031682], GO:0031720, GO:0032182, GO:0032767, GTPase activating protein binding [GO:0032794], GO:0034185, very-low-density lipoprotein particle binding [GO:0034189], inhibin binding [GO:0034711], nodal binding [GO:0038100], co-receptor binding [GO:0039706], histone binding [GO:0042393], identical protein binding [GO:0042802], GO:0042988, ATP-dependent protein binding [GO:0043008], GO:0043221, GO:0043236, proteoglycan binding [GO:0043394], angiostatin binding [GO:0043532], phosphatidylinositol 3-kinase binding [GO:0043548], insulin binding [GO:0043559], insulin receptor substrate binding [GO:0043560], transmembrane transporter binding [GO:0044325], S100 protein binding [GO:0044548], bone sialoprotein binding [GO:0044730], antisigma factor binding [GO:0045152], alpha-catenin binding [GO:0045294], gamma-catenin binding [GO:0045295], GO:0045503, dynein heavy chain binding [GO:0045504], dynein intermediate chain binding [GO:0045505], GO:0045569, SMAD binding [GO:0046332], virion binding [GO:0046790], TAP binding [GO:0046977], tapasin binding [GO:0046980], protein dimerization activity [GO:0046983], calcium-dependent protein binding [GO:0048306], cell adhesion molecule binding [GO:0050839], protein kinase A binding [GO:0051018], GDP-dissociation inhibitor binding [GO:0051021], GO:0051082, protein-folding chaperone binding [GO:0051087], GO:0051219, misfolded protein binding [GO:0051787], dynein light intermediate chain binding [GO:0051959], adiponectin binding [GO:0055100], RBL family protein binding [GO:0061675], importin-alpha family protein binding [GO:0061676], translation elongation factor binding [GO:0061770], proline-rich region binding [GO:0070064], GO:0070097, GO:0070678, sterol-dependent protein binding [GO:0070866], connexin binding [GO:0071253], 14-3-3 protein binding [GO:0071889], endocytic targeting sequence binding [GO:0089710], RHG protein domain binding [GO:0089719], hedgehog family protein binding [GO:0097108], GO:0097110, GO:0097371, GO:0097602, serpin family protein binding [GO:0097655], SOCS family protein binding [GO:0097678], TIMP family protein binding [GO:0098769], FBXO family protein binding [GO:0098770], CNBH domain intrinsic ligand binding [GO:0106151], modification-dependent protein binding [GO:0140030], glycosylated region protein binding [GO:0140081], exogenous protein binding [GO:0140272], cargo receptor ligand activity [GO:0140355], protein antigen binding [GO:1990405], extracellular matrix protein binding [GO:1990430], arrestin family protein binding [GO:1990763], GO:1990935 Also known as: protein amino acid binding, glycoprotein binding Relationships: is a type of GO:0005488